{
  "gene_name": "Palmitoyl-protein thioesterase 1",
  "term_id": "GO:0006897",
  "gene": "UniProtKB:P50897",
  "gene_symbol": "PPT1",
  "term_label": "endocytosis"
}